{
  "gene": "UniProtKB:A6NDV4",
  "term_id": "UNKNOWN:0002",
  "gene_name": "Transmembrane protein 8B",
  "term_label": "Unknown biological process",
  "gene_symbol": "TMEM8B"
}